{
  "gene": "UniProtKB:Q6UXQ8",
  "gene_symbol": "UNQ6190_PRO20217",
  "gene_name": "Putative uncharacterized protein UNQ6190_PRO20217",
  "term_id": "UNKNOWN:0001",
  "term_label": "Unknown molecular function"
}